2-deoxystreptamine metabolic process [GO:1901742] (biological process) Subtypes: 2-deoxystreptamine catabolic process [GO:1901743], 2-deoxystreptamine biosynthetic process [GO:1901744] Definition: The chemical reactions and pathways involving 2-deoxystreptamine. Relationships: is a type of polyol metabolic process [GO:0019751] Also known as: 2-deoxystreptamine metabolism Sources: GOC:TermGenie, GOC:yaf